{
  "term_id": "GO:0003688",
  "gene_symbol": "ORC1",
  "gene": "UniProtKB:Q13415",
  "gene_name": "Origin recognition complex subunit 1",
  "term_label": "DNA replication origin binding"
}